{
  "term_id": "UNKNOWN:0002",
  "gene_symbol": "BLID",
  "gene_name": "BH3-like motif-containing cell death inducer",
  "term_label": "Unknown biological process",
  "gene": "UniProtKB:Q8IZY5"
}